beta-1,4-mannosyltransferase activity [GO:0019187] (molecular function) Definition: Catalysis of the transfer of a mannose residue to an oligosaccharide, forming a beta-(1->4) linkage. References: PMID:8166646 Sources: GOC:mcc Relationships: is a type of mannosyltransferase activity [GO:0000030] Subtypes: chitobiosyldiphosphodolichol beta-mannosyltransferase activity [GO:0004578], glucomannan 4-beta-mannosyltransferase activity [GO:0047259], mannan synthase activity [GO:0051753]